{
  "gene": "UniProtKB:P16949",
  "gene_symbol": "STMN1",
  "term_label": "neuron projection",
  "term_id": "GO:0043005",
  "gene_name": "Stathmin"
}